{
  "gene_name": "Protein dispatched homolog 2",
  "gene": "UniProtKB:A7MBM2",
  "term_id": "UNKNOWN:0001",
  "term_label": "Unknown molecular function",
  "gene_symbol": "DISP2"
}